negative regulation of osteoclast differentiation [GO:0045671] (biological process) Definition: Any process that stops, prevents, or reduces the frequency, rate or extent of osteoclast differentiation. Sources: GOC:go_curators Also known as: down regulation of osteoclast differentiation, down-regulation of osteoclast differentiation, downregulation of osteoclast differentiation, inhibition of osteoclast differentiation Relationships: is a type of negative regulation of myeloid leukocyte differentiation [GO:0002762]; is a type of regulation of osteoclast differentiation [GO:0045670]; negatively regulates osteoclast differentiation [GO:0030316] Subtypes: negative regulation of osteoclast development [GO:2001205]